cellular response to cobalt ion [GO:0071279] (biological process) Sources: GOC:mah Definition: Any process that results in a change in state or activity of a cell (in terms of movement, secretion, enzyme production, gene expression, etc.) as a result of a cobalt ion stimulus. Relationships: is a type of response to cobalt ion [GO:0032025]; is a type of cellular response to metal ion [GO:0071248]